{
  "term_label": "DNA-binding transcription factor activity, RNA polymerase II-specific",
  "gene": "UniProtKB:Q9UIU6",
  "term_id": "GO:0000981",
  "gene_symbol": "SIX4",
  "gene_name": "Homeobox protein SIX4"
}